{
  "term_id": "GO:0005634",
  "gene_name": "Histone H2B type 1-M",
  "term_label": "nucleus",
  "gene": "UniProtKB:Q99879",
  "gene_symbol": "H2BC14"
}